presynapse [GO:0098793] (cellular component) Definition: The part of a synapse that is part of the presynaptic cell. Sources: GOC:dos Relationships: is_a cellular anatomical structure [GO:0110165]; is part of synapse [GO:0045202] Also known as: presynaptic terminal Subtypes: terminal bouton [GO:0043195], GO:0043679